negative regulation of sexual sporulation resulting in formation of a cellular spore [GO:0043942] (biological process) Definition: Any process that stops, prevents, or reduces the frequency, rate or extent of the formation of cellular spores derived from the products of meiosis. Sources: GOC:pamgo_curators Subtypes: negative regulation of oospore formation [GO:0075246], negative regulation of ascospore formation [GO:0075297], negative regulation of zygospore formation [GO:0075300], GO:0075304 Relationships: is a type of negative regulation of sporulation resulting in formation of a cellular spore [GO:0042174]; is a type of regulation of sexual sporulation resulting in formation of a cellular spore [GO:0043940]; is a type of GO:0051447; negatively regulates sexual sporulation resulting in formation of a cellular spore [GO:0043935]